{
  "gene_name": "Ras-related protein Rap-2b",
  "term_label": "GTPase activity",
  "gene_symbol": "RAP2B",
  "term_id": "GO:0003924",
  "gene": "UniProtKB:P61225"
}